{
  "gene_symbol": "TTLL2",
  "term_label": "tubulin binding",
  "gene": "UniProtKB:Q9BWV7",
  "term_id": "GO:0015631",
  "gene_name": "Probable tubulin polyglutamylase TTLL2"
}